septin cytoskeleton organization [GO:0032185] (biological process) Also known as: septin cytoskeleton organisation, septin cytoskeleton organization and biogenesis Subtypes: septin ring organization [GO:0031106], septin collar organization [GO:0140544] Sources: GOC:dph, GOC:jl, GOC:mah Relationships: is a type of cytoskeleton organization [GO:0007010] Definition: A process that is carried out at the cellular level which results in the assembly, arrangement of constituent parts, or disassembly of cytoskeletal structures comprising septin complexes and their associated proteins.